{
  "gene_symbol": "SEC61G",
  "gene_name": "Protein transport protein Sec61 subunit gamma",
  "term_label": "protein transmembrane transporter activity",
  "term_id": "GO:0008320",
  "gene": "UniProtKB:P60059"
}